dGDP metabolic process [GO:0046066] (biological process) Definition: The chemical reactions and pathways involving dGDP, deoxyguanosine diphosphate, (2'-deoxyguanosine 5'-diphosphate). Subtypes: dGDP biosynthetic process [GO:0006185], dGTP biosynthetic process from dGDP [GO:0006187], GO:0046067 Also known as: dGDP metabolism Sources: GOC:go_curators Relationships: is a type of purine deoxyribonucleotide metabolic process [GO:0009151]; is a type of purine deoxyribonucleoside diphosphate metabolic process [GO:0009182]